heart capillary growth [GO:0003248] (biological process) Definition: The increase in heart capillaries that accompanies physiological hypertrophy of cardiac muscle. Relationships: is a type of developmental growth [GO:0048589]; is part of heart growth [GO:0060419]; is part of coronary vasculature development [GO:0060976] Sources: GOC:mtg_heart